{
  "gene_name": "Putative glutamine amidotransferase-like class 1 domain-containing protein 3B, mitochondrial",
  "term_label": "Unknown cellular component",
  "gene_symbol": "GATD3B",
  "gene": "UniProtKB:A0A0B4J2D5",
  "term_id": "UNKNOWN:0003"
}